{
  "term_label": "nucleus",
  "gene_name": "Serine_threonine-protein phosphatase 4 catalytic subunit",
  "gene": "UniProtKB:P60510",
  "term_id": "GO:0005634",
  "gene_symbol": "PPP4C"
}